{
  "term_id": "UNKNOWN:0003",
  "gene_name": "Uncharacterized protein C1orf94",
  "gene": "UniProtKB:Q6P1W5",
  "term_label": "Unknown cellular component",
  "gene_symbol": "C1orf94"
}